{
  "gene": "UniProtKB:Q9H091",
  "term_id": "GO:0042826",
  "term_label": "histone deacetylase binding",
  "gene_symbol": "ZMYND15",
  "gene_name": "Zinc finger MYND domain-containing protein 15"
}